acetylcholine binding [GO:0042166] (molecular function) Sources: GOC:ai Definition: Binding to acetylcholine, an acetic acid ester of the organic base choline that functions as a neurotransmitter, released at the synapses of parasympathetic nerves and at neuromuscular junctions. Relationships: is a type of GO:0043169